{
  "gene_symbol": "CEP170",
  "gene": "UniProtKB:Q5SW79",
  "term_id": "UNKNOWN:0001",
  "term_label": "Unknown molecular function",
  "gene_name": "Centrosomal protein of 170 kDa"
}